primitive hemopoiesis [GO:0060215] (biological process) Definition: A first transient wave of blood cell production that, in vertebrates, gives rise to erythrocytes (red blood cells) and myeloid cells. Also known as: primitive haematopoiesis, primitive haemopoiesis, primitive hematopoiesis Relationships: is a type of embryonic hemopoiesis [GO:0035162] References: PMID:15378083, PMID:15617691 Sources: GOC:bf, GOC:dph